protein catabolic process at postsynapse [GO:0140249] (biological process) Note: Note that this term was created for the SynGO project, and will be obsoleted when the SynGO annotations are made in Noctua. Definition: The chemical reactions and pathways resulting in the breakdown of a protein at a postsynapse. Relationships: is a type of GO:0140246; occurs in postsynapse [GO:0098794] References: PMID:17062563